{
  "gene": "UniProtKB:Q99986",
  "gene_name": "Serine_threonine-protein kinase VRK1",
  "term_label": "cytoplasm",
  "gene_symbol": "VRK1",
  "term_id": "GO:0005737"
}